{
  "term_id": "UNKNOWN:0003",
  "gene_symbol": "EXOC1L",
  "term_label": "Unknown cellular component",
  "gene_name": "Exocyst complex component 1-like",
  "gene": "UniProtKB:A0A1B0GW35"
}